fluorothreonine transaldolase activity [GO:0033806] (molecular function) Definition: Catalysis of the reaction: L-threonine + fluoroacetaldehyde = acetaldehyde + 4-fluoro-L-threonine. Also known as: fluoroacetaldehyde:L-threonine aldehydetransferase activity Relationships: is a type of GO:0016744 Sources: RHEA:11748